{
  "term_label": "nBAF complex",
  "term_id": "GO:0071565",
  "gene": "UniProtKB:Q92782",
  "gene_name": "Zinc finger protein neuro-d4",
  "gene_symbol": "DPF1"
}